{
  "term_label": "plasma membrane",
  "gene_name": "Retinoic acid-induced protein 3",
  "term_id": "GO:0005886",
  "gene": "UniProtKB:Q8NFJ5",
  "gene_symbol": "GPRC5A"
}